{
  "gene_symbol": "TRBV6-9",
  "gene_name": "T cell receptor beta variable 6-9",
  "term_label": "Unknown molecular function",
  "gene": "UniProtKB:A0A0J9YX75",
  "term_id": "UNKNOWN:0001"
}